{
  "gene_name": "C4b-binding protein beta chain",
  "gene": "UniProtKB:P20851",
  "term_label": "Unknown cellular component",
  "term_id": "UNKNOWN:0003",
  "gene_symbol": "C4BPB"
}